branched duct epithelial cell fate determination, open tracheal system [GO:0046845] (biological process) Definition: Allocation of a set number of cells to each primary branch in an open tracheal system, prior to the onset of cell migration. This establishes different domains of cells within the tracheal placode. References: PMID:10684581 Sources: GOC:mtg_sensu Also known as: branch cell fate determination Relationships: is a type of GO:0001709; is part of open tracheal system development [GO:0007424]